(S)-tetrahydroprotoberberine N-methyltransferase activity [GO:0030782] (molecular function) Definition: Catalysis of the reaction: an (S)-7,8,13,14-tetrahydroprotoberberine + S-adenosyl-L-methionine = an (S)-cis-N-methyl-7,8,13,14-tetrahydroprotoberberine + S-adenosyl-L-homocysteine. Sources: RHEA:76067 Also known as: S-adenosyl-L-methionine:(S)-7,8,13,14-tetrahydroprotoberberine cis-N-methyltransferase activity, tetrahydroprotoberberine cis-N-methyltransferase activity Relationships: is a type of GO:0008757